{
  "term_label": "mucus secretion",
  "term_id": "GO:0070254",
  "gene_name": "Vesicle-associated membrane protein 8",
  "gene": "UniProtKB:Q9BV40",
  "gene_symbol": "VAMP8"
}